{
  "gene": "UniProtKB:Q16581",
  "gene_symbol": "C3AR1",
  "gene_name": "C3a anaphylatoxin chemotactic receptor",
  "term_id": "GO:0006954",
  "term_label": "inflammatory response"
}